myricetin 3'-O-methyltransferase activity [GO:0033799] (molecular function) Relationships: is a type of O-methyltransferase activity [GO:0008171]; is a type of GO:0008757 Sources: RHEA:25629 Also known as: CrCOMT2, S-adenosyl-L-methionine:myricetin O-methyltransferase activity, flavonoid 3',5'-O-dimethyltransferase activity, myricetin 3-O-methyltransferase activity Definition: Catalysis of the reaction: S-adenosyl-L-methionine + myricetin = S-adenosyl-L-homocysteine + laricitrin.